{
  "gene": "UniProtKB:O15405",
  "gene_name": "TOX high mobility group box family member 3",
  "gene_symbol": "TOX3",
  "term_label": "nucleus",
  "term_id": "GO:0005634"
}